{
  "term_label": "Unknown biological process",
  "term_id": "UNKNOWN:0002",
  "gene_name": "Very long-chain specific acyl-CoA dehydrogenase, mitochondrial",
  "gene": "UniProtKB:P49748",
  "gene_symbol": "ACADVL"
}